{
  "term_label": "nucleus",
  "gene_symbol": "CCND2",
  "gene_name": "G1_S-specific cyclin-D2",
  "gene": "UniProtKB:P30279",
  "term_id": "GO:0005634"
}